estrous cycle phase [GO:0060206] (biological process) Sources: GOC:dph Relationships: is a type of GO:0044848 Note: Note that this term should not be used for direct annotation. If you are trying to make an annotation to x phase, it is likely that the correct annotation is 'regulation of x/y phase transition' or to a process which occurs during the reported phase. To capture the phase when a specific location or process is observed, the phase term can be used in an annotation extension (PMID:24885854) applied to a cellular component term (with the relation exists_during) or a biological process term (with the relation happens_during). Subtypes: diestrus [GO:0060207], proestrus [GO:0060208], estrus [GO:0060209], metestrus [GO:0060210] Definition: The progression of physiological phases, occurring in the endometrium during the estrous cycle that recur at regular intervals during the reproductive years. The estrous cycle is an ovulation cycle where the endometrium is resorbed if pregnancy does not occur.